host cell junction [GO:0044156] (cellular component) Definition: A plasma membrane part that forms a specialized region of connection between two host cells or between a host cell and the host extracellular matrix. At a host cell junction, anchoring proteins extend through the host plasma membrane to link cytoskeletal proteins in one cell to cytoskeletal proteins in neighboring cells or to proteins in the extracellular matrix. Sources: GOC:rph Relationships: is a type of host cell part [GO:0033643]; is part of GO:0020002 Subtypes: GO:0044219